protein-lysine lysyltransferase activity [GO:0052868] (MF) References: PMID:20729861 Relationships: is a type of aminoacyltransferase activity [GO:0016755]; is_a GO:0140096 Definition: Catalysis of the reaction: protein-lysine + protein-lysine = protein N6-(lysyl)-L-lysine + protein. This reaction is the addition of lysine group from one protein to a lysine residue in a second protein, producing N6-(lysyl)-L-lysine.